negative regulation of melanization defense response [GO:0035009] (biological process) Subtypes: negative regulation melanotic encapsulation of foreign target [GO:0140540] Definition: Any process that reduces the rate or extent of the melanization defense response. This regulation is critical to limit melanization to the site of injury or infection. References: PMID:12408809 Sources: GOC:bf Also known as: down regulation of melanization defense response, down-regulation of melanization defense response, downregulation of melanization defense response, negative regulation of melanization defence response, inhibition of melanization defense response Relationships: is a type of negative regulation of metabolic process [GO:0009892]; is a type of regulation of melanization defense response [GO:0035007]; is a type of negative regulation of innate immune response [GO:0045824]; negatively regulates melanization defense response [GO:0035006]